{
  "term_id": "GO:0009408",
  "gene_name": "Heat shock protein beta-1",
  "gene": "UniProtKB:P04792",
  "gene_symbol": "HSPB1",
  "term_label": "response to heat"
}